{
  "term_label": "positive regulation of cell migration",
  "gene_name": "C-C motif chemokine 7",
  "gene": "UniProtKB:P80098",
  "term_id": "GO:0030335",
  "gene_symbol": "CCL7"
}